photosynthetic electron transport in photosystem II [GO:0009772] (BP) Relationships: is a type of GO:0009767 Definition: A photosynthetic electron transport chain in which electrons move from the primary electron acceptor (Quinone, Q) through a chain of electron transport molecules in the thylakoid membrane until they reach the ultimate electron acceptor of Photosystem II, which is plastocyanin (PC). The electron is then passed to the P700 chlorophyll a molecules of the reaction centre of photosystem I. Sources: GOC:jid, ISBN:0716731363, ISBN:0816017360